{
  "gene_name": "Alpha-(1,3)-fucosyltransferase 4",
  "term_id": "UNKNOWN:0003",
  "term_label": "Unknown cellular component",
  "gene": "UniProtKB:P22083",
  "gene_symbol": "FUT4"
}